apoptotic process involved in tube lumen cavitation [GO:0060609] (biological process) Definition: Any apoptotic process that contributes to the hollowing out of an epithelial rod or cord to form the central hole in a tube. Subtypes: apoptotic process involved in salivary gland cavitation [GO:0060663] Sources: GOC:dph, GOC:mtg_apoptosis Also known as: apoptosis involved in tube lumen cavitation Relationships: is a type of apoptotic process involved in morphogenesis [GO:0060561]; is part of tube lumen cavitation [GO:0060605]